{
  "term_id": "GO:1990259",
  "term_label": "histone H2AQ104 methyltransferase activity",
  "gene": "UniProtKB:P22087",
  "gene_symbol": "FBL",
  "gene_name": "rRNA 2'-O-methyltransferase fibrillarin"
}